{
  "gene_symbol": "NKX6-2",
  "term_id": "GO:0000981",
  "term_label": "DNA-binding transcription factor activity, RNA polymerase II-specific",
  "gene_name": "Homeobox protein Nkx-6.2",
  "gene": "UniProtKB:Q9C056"
}